meristemoid mother cell division [GO:0010443] (biological process) Relationships: is a type of cytokinesis by cell plate formation [GO:0000911]; is part of stomatal lineage progression [GO:0010440] Also known as: meristemoid division Sources: GOC:expert_db, GOC:tb Definition: The asymmetric cell division by which a meristemoid mother cells (MMC) give rise to a meristemoid and another cell. The other cell may itself become a MMC or may generate an epidermal cell. Any cell that undergoes this type of division is a MMC.